{
  "term_id": "UNKNOWN:0002",
  "term_label": "Unknown biological process",
  "gene_name": "Late cornified envelope protein 1D",
  "gene_symbol": "LCE1D",
  "gene": "UniProtKB:Q5T752"
}